{
  "term_id": "UNKNOWN:0002",
  "gene_name": "Kelch domain-containing protein 9",
  "gene_symbol": "KLHDC9",
  "gene": "UniProtKB:Q8NEP7",
  "term_label": "Unknown biological process"
}